{
  "term_label": "Unknown cellular component",
  "term_id": "UNKNOWN:0003",
  "gene_name": "Transmembrane protein 144",
  "gene": "UniProtKB:Q7Z5S9",
  "gene_symbol": "TMEM144"
}